{
  "term_id": "GO:0005829",
  "gene_name": "Ubiquitin carboxyl-terminal hydrolase 17-like protein 20",
  "term_label": "cytosol",
  "gene_symbol": "USP17L20",
  "gene": "UniProtKB:D6RJB6"
}